unmodified histone reader activity [GO:0140063] (molecular function) Relationships: is a type of histone reader activity [GO:0140566] Note: Curator note: To annotate the specific histone recognized, use 'has input' extension. Definition: A histone reader that specifically binds either to an unmodified histone. Sources: GOC:pg